{
  "gene": "UniProtKB:Q8NGJ4",
  "gene_name": "Olfactory receptor 52E2",
  "gene_symbol": "OR52E2",
  "term_id": "UNKNOWN:0002",
  "term_label": "Unknown biological process"
}